astrocyte cell migration [GO:0043615] (biological process) Definition: The orderly movement of an astrocyte, a class of large neuroglial (macroglial) cells in the central nervous system, the largest and most numerous neuroglial cells in the brain and spinal cord. Sources: CL:0000127, GOC:go_curators Also known as: astrocyte migration, astrocytic glial cell migration Relationships: is a type of glial cell migration [GO:0008347] Subtypes: telencephalon astrocyte cell migration [GO:0022031], astrocyte chemotaxis [GO:0035700]